negative regulation of natural killer cell cytokine production [GO:0002728] (biological process) Definition: Any process that stops, prevents, or reduces the frequency, rate, or extent of natural killer cell cytokine production. Sources: GOC:add Also known as: down regulation of natural killer cell cytokine production, down-regulation of natural killer cell cytokine production, downregulation of natural killer cell cytokine production, negative regulation of NK cell cytokine production, inhibition of natural killer cell cytokine production Relationships: is a type of GO:0002716; is a type of negative regulation of cytokine production involved in immune response [GO:0002719]; is a type of regulation of natural killer cell cytokine production [GO:0002727]; negatively regulates natural killer cell cytokine production [GO:0002370]